paranodal junction maintenance [GO:1990227] (biological process) References: PMID:24011083 Sources: GOC:pr Also known as: axoglial septate junction maintenance, paranodal axoglial junction maintenance, paranodal septate maintenance Relationships: is a type of GO:0045217 Definition: The maintenance of a paranodal junction, a highly specialized cell-cell junction found in vertebrates, which forms between a neuron and a glial cell, and has structural similarity to Drosophila septate junctions. A paranodal junction flanks the node of Ranvier in myelinated nerve, electrically isolates the myelinated from unmyelinated nerve segments, and physically separates the voltage-gated sodium channels at the node from the cluster of potassium channels underneath the myelin sheath.